{
  "term_id": "UNKNOWN:0003",
  "gene_symbol": "Q6ZRX8",
  "gene_name": "Putative uncharacterized protein FLJ45999",
  "gene": "UniProtKB:Q6ZRX8",
  "term_label": "Unknown cellular component"
}